{
  "gene_symbol": "PCDHB18P",
  "term_id": "GO:0050839",
  "term_label": "cell adhesion molecule binding",
  "gene_name": "Putative protocadherin beta-18",
  "gene": "UniProtKB:Q96TA0"
}